{
  "term_label": "Unknown cellular component",
  "gene_name": "Galanin-like peptide",
  "gene": "UniProtKB:Q9UBC7",
  "gene_symbol": "GALP",
  "term_id": "UNKNOWN:0003"
}